positive regulation of starch catabolic process [GO:2000883] (biological process) Definition: Any process that activates or increases the frequency, rate or extent of starch catabolic process. Relationships: is_a positive regulation of catabolic process [GO:0009896]; is a type of positive regulation of macromolecule metabolic process [GO:0010604]; is a type of GO:0045913; is a type of GO:2000881; positively regulates starch catabolic process [GO:0005983] Also known as: positive regulation of starch breakdown, positive regulation of starch catabolism, positive regulation of starch degradation Sources: GOC:obol Subtypes: positive regulation of amylopectin catabolic process [GO:2000947]